{
  "term_label": "ABC-type xenobiotic transporter activity",
  "gene_symbol": "ABCC2",
  "gene_name": "ATP-binding cassette sub-family C member 2",
  "term_id": "GO:0008559",
  "gene": "UniProtKB:Q92887"
}